regulation of interleukin-33 production [GO:0150127] (biological process) Definition: Any process that modulates the frequency, rate or extent of interleukin-33 production. Also known as: regulation of interleukin-33 biosynthetic process, regulation of interleukin-33 secretion Subtypes: negative regulation of interleukin-33 production [GO:0150128], GO:0150129 Relationships: is a type of regulation of cytokine production [GO:0001817]; regulates interleukin-33 production [GO:0072639] References: PMID:29778524 Sources: GOC:aruk